piperitol synthase activity [GO:0102915] (molecular function) Definition: Catalysis of the reaction: H+ + (+)-pinoresinol + NADPH + O2 = (+)-piperitol + NADP + 2 H2O. Relationships: is a type of GO:0016709 References: PMID:16785429 Sources: EC:1.14.19.74